positive regulation of fatty acid beta-oxidation by serotonin receptor signaling pathway [GO:1904123] (biological process) References: PMID:24120942 Sources: GOC:TermGenie, GOC:dph, GOC:kmv, GO_REF:0000063 Also known as: up regulation of fatty acid beta-oxidation by serotonin receptor signaling pathway, up-regulation of fatty acid beta-oxidation by serotonin receptor signaling pathway, upregulation of fatty acid beta-oxidation by serotonin receptor signaling pathway, activation of fatty acid beta-oxidation by serotonin receptor signaling pathway, stimulation of fatty acid beta-oxidation by serotonin receptor signaling pathway Definition: A serotonin receptor signaling pathway that results in positive regulation of fatty acid beta-oxidation. Relationships: is a type of serotonin receptor signaling pathway [GO:0007210]; is a type of positive regulation of fatty acid beta-oxidation [GO:0032000]